{
  "term_id": "GO:0006954",
  "gene": "UniProtKB:P42830",
  "term_label": "inflammatory response",
  "gene_symbol": "CXCL5",
  "gene_name": "C-X-C motif chemokine 5"
}